L-threonine catabolic process to glycine [GO:0019518] (biological process) Definition: The chemical reactions and pathways resulting in the breakdown of L-threonine (the L-enantiomer of 2-amino-3-hydroxybutyric acid) to form 2-amino-3-oxobutanoate, which is subsequently converted to glycine. Also known as: threonine catabolic process to glycine, L-threonine breakdown to glycine, L-threonine catabolism to glycine, L-threonine degradation to glycine, glycine biosynthetic process from L-threonine, L-threonine catabolic process to pyruvate References: PMID:728468 Sources: GOC:bf, GOC:mah, MetaCyc:THREONINE-DEG2-PWY Relationships: is a type of glycine biosynthetic process [GO:0006545]; is a type of L-threonine catabolic process [GO:0006567]